{
  "gene_name": "FRAS1-related extracellular matrix protein 3",
  "term_id": "UNKNOWN:0001",
  "gene": "UniProtKB:P0C091",
  "gene_symbol": "FREM3",
  "term_label": "Unknown molecular function"
}